{
  "term_id": "GO:0031012",
  "gene_name": "Protein disulfide isomerase CRELD1",
  "gene_symbol": "CRELD1",
  "gene": "UniProtKB:Q96HD1",
  "term_label": "extracellular matrix"
}